{
  "term_label": "negative regulation of protein localization to microtubule",
  "term_id": "GO:1902817",
  "gene": "UniProtKB:Q96GS6",
  "gene_name": "Alpha_beta hydrolase domain-containing protein 17A",
  "gene_symbol": "ABHD17A"
}